parathion catabolic process [GO:0019339] (biological process) Definition: The chemical reactions and pathways resulting in the breakdown of parathion, a highly toxic organophosphate compound. Degradation of parathion by sunlight or liver enzymes can result in the formation of the active compound paraoxon which interferes with the nervous system through cholinesterase inhibition. Sources: MetaCyc:PARATHION-DEGRADATION-PWY Also known as: parathion breakdown, parathion catabolism, parathion degradation Relationships: is a type of phosphate-containing compound metabolic process [GO:0006796]; is a type of GO:0044273; is a type of organophosphate catabolic process [GO:0046434]